{
  "gene_name": "Ras-related C3 botulinum toxin substrate 3",
  "gene": "UniProtKB:P60763",
  "term_label": "GTP binding",
  "gene_symbol": "RAC3",
  "term_id": "GO:0005525"
}